arabidiol synthase activity [GO:0034075] (molecular function) Relationships: is a type of oxidosqualene cyclase activity [GO:0031559] References: PMID:16774269, PMID:17474751 Sources: GOC:cb Definition: Catalysis of the reaction: oxidosqualene + H2O = arabidiol ((13R,14R,17E)-malabarica-17,21-diene-3beta,14-diol).